peroxynitrite reductase activity [GO:0072541] (molecular function) Relationships: is a type of peroxidase activity [GO:0004601] Definition: Catalysis of the reaction: [protein]-dithiol + ONOO- = [protein]-disulfide + NO2- + H2O. Note: Note that this activity is usually associated in vivo with an NADPH-dependent disulfide reductase activity, so that catalysis of the reduction of peroxynitrite to nitrite involves the possible creation of oxygen or water, using NADPH as reduction equivalent. Also known as: peroxynitritase activity References: PMID:11001062 Sources: GOC:rs